{
  "gene_symbol": "PUS3",
  "term_id": "GO:0005737",
  "term_label": "cytoplasm",
  "gene_name": "tRNA pseudouridine(38_39) synthase",
  "gene": "UniProtKB:Q9BZE2"
}